{
  "gene_name": "Slit homolog 1 protein",
  "term_label": "heparin binding",
  "gene": "UniProtKB:O75093",
  "term_id": "GO:0008201",
  "gene_symbol": "SLIT1"
}